{
  "gene_name": "Transmembrane protein 132B",
  "term_label": "Unknown biological process",
  "term_id": "UNKNOWN:0002",
  "gene_symbol": "TMEM132B",
  "gene": "UniProtKB:Q14DG7"
}